endothelial cell differentiation [GO:0045446] (biological process) Regulation: regulated by regulation of endothelial cell differentiation [GO:0045601]; negatively regulated by negative regulation of endothelial cell differentiation [GO:0045602]; positively regulated by positive regulation of endothelial cell differentiation [GO:0045603] Subtypes: GO:0003348, lymphatic endothelial cell differentiation [GO:0060836], blood vessel endothelial cell differentiation [GO:0060837] Sources: CL:0000115, GOC:go_curators Relationships: is a type of epithelial cell differentiation [GO:0030855]; is part of endothelium development [GO:0003158] Definition: The process in which a mesodermal, bone marrow or neural crest cell acquires specialized features of an endothelial cell, a thin flattened cell. A layer of such cells lines the inside surfaces of body cavities, blood vessels, and lymph vessels, making up the endothelium.